imidazole N-acetyltransferase activity [GO:0047716] (molecular function) Also known as: acetyl-CoA:imidazole N-acetyltransferase activity, imidazole acetylase activity, imidazole acetyltransferase activity Relationships: is a type of N-acetyltransferase activity [GO:0008080] Definition: Catalysis of the reaction: 1H-imidazole + acetyl-CoA = N-acetylimidazole + CoA. Sources: EC:2.3.1.2, RHEA:15813